GDP-D-mannose biosynthetic process from fructose-6-phosphate [GO:0061729] (biological process) References: PMID:16339137 Sources: GOC:dph Relationships: is a type of GDP-mannose biosynthetic process [GO:0009298]; has part mannose-6-phosphate isomerase activity [GO:0004476] Definition: The chemical reactions and pathways resulting in the formation of GDP-D-mannose from D-fructose-6-phosphate. Also known as: GDP-mannose biosynthetic process from fructose-6-phosphate, GDP-mannose biosynthetic process from glucose